{
  "gene_symbol": "RPS11",
  "gene": "UniProtKB:P62280",
  "term_label": "Unknown biological process",
  "term_id": "UNKNOWN:0002",
  "gene_name": "Small ribosomal subunit protein uS17"
}